{
  "term_id": "UNKNOWN:0002",
  "gene": "UniProtKB:A8MQ11",
  "gene_name": "Postmeiotic segregation increased 2-like protein 5",
  "term_label": "Unknown biological process",
  "gene_symbol": "PMS2P5"
}